ent-kaurene synthase activity [GO:0009899] (molecular function) Sources: EC:4.2.3.19, RHEA:22220 Relationships: is_a terpene synthase activity [GO:0010333] Also known as: ent-kaurene synthase B activity, ent-kaurene synthetase B activity, ent-copalyl-diphosphate diphosphate-lyase (cyclizing), ent-copalyl-diphosphate diphosphate-lyase (cyclizing, ent-kaurene-forming) Definition: Catalysis of the reaction: ent-copalyl diphosphate = ent-kaur-16-ene + diphosphate.